{
  "gene": "UniProtKB:Q9UHJ6",
  "term_id": "GO:0005829",
  "gene_symbol": "SHPK",
  "gene_name": "Sedoheptulokinase",
  "term_label": "cytosol"
}